{
  "gene_name": "Cyclin-dependent kinase inhibitor 1",
  "gene": "UniProtKB:P38936",
  "gene_symbol": "CDKN1A",
  "term_id": "GO:0004860",
  "term_label": "protein kinase inhibitor activity"
}